{
  "term_label": "endoplasmic reticulum to Golgi vesicle-mediated transport",
  "gene_symbol": "CTAGE1",
  "term_id": "GO:0006888",
  "gene_name": "cTAGE family member 2",
  "gene": "UniProtKB:Q96RT6"
}